{
  "gene_name": "Zinc finger protein 677",
  "gene": "UniProtKB:Q86XU0",
  "term_label": "DNA-binding transcription factor activity, RNA polymerase II-specific",
  "gene_symbol": "ZNF677",
  "term_id": "GO:0000981"
}